{
  "gene_symbol": "PSMB2",
  "gene": "UniProtKB:P49721",
  "gene_name": "Proteasome subunit beta type-2",
  "term_id": "GO:0043161",
  "term_label": "proteasome-mediated ubiquitin-dependent protein catabolic process"
}